{
  "gene_name": "Tripartite motif-containing protein 77",
  "gene_symbol": "TRIM77",
  "gene": "UniProtKB:I1YAP6",
  "term_label": "innate immune response",
  "term_id": "GO:0045087"
}